tryptophanyl-tRNA aminoacylation [GO:0006436] (biological process) Subtypes: mitochondrial tryptophanyl-tRNA aminoacylation [GO:0070183] Relationships: is a type of tRNA aminoacylation for protein translation [GO:0006418] Definition: The process of coupling tryptophan to tryptophanyl-tRNA, catalyzed by tryptophanyl-tRNA synthetase. The tryptophanyl-tRNA synthetase is a class-I synthetase. The activated amino acid is transferred to the 2'-OH group of a tryptophan-accetping tRNA. The 2'-O-aminoacyl-tRNA will ultimately migrate to the 3' position via transesterification. Sources: GOC:mcc, ISBN:0716730510